{
  "term_id": "GO:0005739",
  "gene": "UniProtKB:P23786",
  "gene_name": "Carnitine O-palmitoyltransferase 2, mitochondrial",
  "term_label": "mitochondrion",
  "gene_symbol": "CPT2"
}